{
  "gene_name": "Rab GDP dissociation inhibitor alpha",
  "term_id": "GO:0005829",
  "term_label": "cytosol",
  "gene_symbol": "GDI1",
  "gene": "UniProtKB:P31150"
}